{
  "gene": "UniProtKB:Q5VY43",
  "term_id": "UNKNOWN:0001",
  "term_label": "Unknown molecular function",
  "gene_name": "Platelet endothelial aggregation receptor 1",
  "gene_symbol": "PEAR1"
}